{
  "term_label": "structural constituent of cytoskeleton",
  "term_id": "GO:0005200",
  "gene_name": "Tubulin beta-2A chain",
  "gene_symbol": "TUBB2A",
  "gene": "UniProtKB:Q13885"
}